{
  "term_id": "GO:0000977",
  "gene_name": "Homeobox protein Hox-B8",
  "gene_symbol": "HOXB8",
  "gene": "UniProtKB:P17481",
  "term_label": "RNA polymerase II transcription regulatory region sequence-specific DNA binding"
}